{
  "term_label": "Unknown molecular function",
  "term_id": "UNKNOWN:0001",
  "gene_name": "F-box_WD repeat-containing protein 10",
  "gene_symbol": "FBXW10",
  "gene": "UniProtKB:Q5XX13"
}